positive regulation of reactive oxygen species metabolic process [GO:2000379] (biological process) Relationships: is a type of GO:0009893; is a type of GO:2000377; positively regulates reactive oxygen species metabolic process [GO:0072593] Subtypes: positive regulation of superoxide anion generation [GO:0032930], positive regulation of hydrogen peroxide catabolic process [GO:1903285], positive regulation of reactive oxygen species biosynthetic process [GO:1903428], positive regulation of removal of superoxide radicals [GO:1904833] Definition: Any process that activates or increases the frequency, rate or extent of reactive oxygen species metabolic process. Also known as: positive regulation of ROS metabolic process, positive regulation of reactive oxygen species metabolism Sources: GOC:mah